{
  "term_id": "GO:0005923",
  "term_label": "bicellular tight junction",
  "gene_symbol": "CLDN19",
  "gene_name": "Claudin-19",
  "gene": "UniProtKB:Q8N6F1"
}